psilocybin biosynthetic process [GO:0140380] (biological process) Relationships: is_a L-tryptophan metabolic process [GO:0006568]; is a type of phosphate-containing compound metabolic process [GO:0006796]; is a type of indole alkaloid biosynthetic process [GO:0035835]; is a type of indole-containing compound biosynthetic process [GO:0042435]; is a type of mycotoxin biosynthetic process [GO:0043386]; is a type of organophosphate biosynthetic process [GO:0090407]; has part L-tryptophan decarboxylase activity [GO:0036469]; has part 4-hydroxytryptamine 4-phosphate methyltransferase activity [GO:0140381]; has part GO:0140382; has part 4-hydroxytryptamine kinase activity [GO:0140383] References: PMID:28763571 Definition: The chemical reactions and pathways resulting in the formation of psilocybin, a psychotropic tryptamine-derived natural product.